{
  "gene": "UniProtKB:Q8N5F7",
  "gene_name": "NF-kappa-B-activating protein",
  "gene_symbol": "NKAP",
  "term_label": "nucleus",
  "term_id": "GO:0005634"
}